{
  "term_label": "extracellular space",
  "term_id": "GO:0005615",
  "gene_symbol": "CPB1",
  "gene_name": "Carboxypeptidase B",
  "gene": "UniProtKB:P15086"
}